inhibitory MHC class I receptor activity [GO:0032396] (MF) Subtypes: HLA-A specific inhibitory MHC class I receptor activity [GO:0030107], GO:0030109, HLA-C specific inhibitory MHC class I receptor activity [GO:0030110] Definition: Combining with a MHC class I protein complex to mediate signaling that inhibits activation of a lymphocyte. References: PMID:11858820, PMID:9368779, PMID:9597134 Sources: GOC:add Relationships: is a type of MHC class I receptor activity [GO:0032393]